{
  "term_label": "cytosol",
  "gene_name": "All-trans-retinol dehydrogenase [NAD(+)] ADH1B",
  "gene": "UniProtKB:P00325",
  "gene_symbol": "ADH1B",
  "term_id": "GO:0005829"
}